macrophage cytokine production [GO:0010934] (biological process) Sources: GOC:BHF, GOC:dph, GOC:rl, GOC:tb Definition: The appearance of a macrophage cytokine due to biosynthesis or secretion following a cellular stimulus, resulting in an increase in its intracellular or extracellular levels. Regulation: RO_0002211 by regulation of macrophage cytokine production [GO:0010935]; negatively regulated by negative regulation of macrophage cytokine production [GO:0010936]; positively regulated by positive regulation of macrophage cytokine production [GO:0060907] Note: Note that this term is in the subset of terms that should not be used for direct gene product annotation. Instead, select one of the 'regulation' children terms. Relationships: is a type of myeloid leukocyte cytokine production [GO:0061082]